{
  "term_label": "transcription-dependent tethering of RNA polymerase II gene DNA at nuclear periphery",
  "gene_name": "mRNA export factor RAE1",
  "gene_symbol": "RAE1",
  "term_id": "GO:0000972",
  "gene": "UniProtKB:P78406"
}